{
  "term_label": "Unknown molecular function",
  "gene": "UniProtKB:Q96GK7",
  "gene_name": "Fumarylacetoacetate hydrolase domain-containing protein 2A",
  "gene_symbol": "FAHD2A",
  "term_id": "UNKNOWN:0001"
}